{
  "gene_symbol": "CFAP300",
  "gene": "UniProtKB:Q9BRQ4",
  "term_id": "UNKNOWN:0002",
  "term_label": "Unknown biological process",
  "gene_name": "Cilia- and flagella-associated protein 300"
}